hexose mediated signaling [GO:0009757] (biological process) Definition: The series of molecular signals mediated by the detection of hexose. Sources: GOC:sm Also known as: hexose mediated signalling Relationships: is a type of sugar mediated signaling pathway [GO:0010182]; is part of cellular response to hexose stimulus [GO:0071331] Subtypes: hexokinase-dependent signaling [GO:0009747], hexokinase-independent signaling [GO:0009748], GO:0010255